{
  "term_label": "mechanosensitive monoatomic ion channel activity",
  "term_id": "GO:0008381",
  "gene": "UniProtKB:Q6UXY8",
  "gene_symbol": "TMC5",
  "gene_name": "Transmembrane channel-like protein 5"
}